positive regulation of interleukin-3 production [GO:0032752] (biological process) Sources: GOC:mah Relationships: is a type of positive regulation of cytokine production [GO:0001819]; is a type of regulation of interleukin-3 production [GO:0032672]; positively regulates interleukin-3 production [GO:0032632] Also known as: positive regulation of IL-3 production, up regulation of interleukin-3 production, up-regulation of interleukin-3 production, upregulation of interleukin-3 production, activation of interleukin-3 production, positive regulation of interleukin-3 biosynthetic process, stimulation of interleukin-3 production Definition: Any process that activates or increases the frequency, rate, or extent of interleukin-3 production.